transposable element silencing [GO:0010526] (biological process) References: PMID:32823517 Sources: GOC:dph, GOC:tb Subtypes: transposable element silencing by heterochromatin formation [GO:0141005], transposable element silencing by mRNA destabilization [GO:0141008] Definition: Any process that decreases the frequency, rate or extent of transposable element expression. Includes both DNA transposons and retrotransposons. Relationships: is a type of GO:0010629; negatively regulates retrotransposition [GO:0032197] Also known as: negative regulation of transposition, RNA-mediated, retrotransposon silencing